cellular response to ozone [GO:0071457] (biological process) Relationships: is a type of response to ozone [GO:0010193]; is a type of GO:0034614 Sources: GOC:mah Definition: Any process that results in a change in state or activity of a cell (in terms of movement, secretion, enzyme production, gene expression, etc.) as a result of a ozone stimulus.